{
  "term_label": "lipid catabolic process",
  "gene_name": "Lipase member I",
  "gene_symbol": "LIPI",
  "term_id": "GO:0016042",
  "gene": "UniProtKB:Q6XZB0"
}